regulation of complement activation, classical pathway [GO:0030450] (biological process) Sources: GOC:go_curators Relationships: is a type of regulation of humoral immune response mediated by circulating immunoglobulin [GO:0002923]; is a type of GO:0030449; regulates complement activation, classical pathway [GO:0006958] Subtypes: GO:0045959, positive regulation of complement activation, classical pathway [GO:0045960] Also known as: regulation of complement cascade, classical pathway Definition: Any process that modulates the frequency, rate or extent of the classical pathway of complement activation.